{
  "gene": "UniProtKB:Q8IZ16",
  "term_id": "UNKNOWN:0002",
  "term_label": "Unknown biological process",
  "gene_symbol": "SPACDR",
  "gene_name": "Sperm acrosome developmental regulator"
}